{
  "term_id": "GO:0034122",
  "gene": "UniProtKB:Q9UBC1",
  "gene_name": "NF-kappa-B inhibitor-like protein 1",
  "gene_symbol": "NFKBIL1",
  "term_label": "negative regulation of toll-like receptor signaling pathway"
}